pantoate-beta-alanine ligase activity [GO:0004592] (molecular function) Definition: Catalysis of the reaction: ATP + (R)-pantoate + beta-alanine = AMP + diphosphate + (R)-pantothenate. Also known as: (R)-pantoate:beta-alanine ligase (AMP-forming), D-pantoate:beta-alanine ligase (AMP-forming), pantoate-activating enzyme activity, pantoic-activating enzyme activity, pantothenate synthetase activity Relationships: is a type of acid-amino acid ligase activity [GO:0016881] Sources: EC:6.3.2.1